vestibulocochlear nerve formation [GO:0021650] (biological process) Relationships: is a type of cranial nerve formation [GO:0021603]; is part of vestibulocochlear nerve morphogenesis [GO:0021648] Also known as: CN VII formation Sources: GOC:cls, GOC:dgh, GOC:dph, GOC:jid, GO_REF:0000021 Definition: The process that gives rise to the vestibulocochlear nerve. This process pertains to the initial formation of a structure from unspecified parts. This sensory nerve innervates the membranous labyrinth of the inner ear. The vestibular branch innervates the vestibular apparatus that senses head position changes relative to gravity. The auditory branch innervates the cochlear duct, which is connected to the three bony ossicles which transduce sound waves into fluid movement in the cochlea.